{
  "gene": "UniProtKB:Q99650",
  "term_label": "cytokine-mediated signaling pathway",
  "gene_symbol": "OSMR",
  "gene_name": "Oncostatin-M-specific receptor subunit beta",
  "term_id": "GO:0019221"
}